{
  "gene": "UniProtKB:Q7Z3I7",
  "term_id": "GO:0001227",
  "term_label": "DNA-binding transcription repressor activity, RNA polymerase II-specific",
  "gene_symbol": "ZNF572",
  "gene_name": "Zinc finger protein 572"
}